{
  "gene_symbol": "B3GNT2",
  "gene": "UniProtKB:Q9NY97",
  "gene_name": "N-acetyllactosaminide beta-1,3-N-acetylglucosaminyltransferase 2",
  "term_label": "poly-N-acetyllactosamine biosynthetic process",
  "term_id": "GO:0030311"
}